{
  "gene_name": "Programmed cell death protein 6",
  "gene": "UniProtKB:O75340",
  "term_id": "UNKNOWN:0001",
  "term_label": "Unknown molecular function",
  "gene_symbol": "PDCD6"
}